{
  "gene_name": "Cyclin-dependent kinase 2",
  "term_label": "cytoplasm",
  "gene_symbol": "CDK2",
  "term_id": "GO:0005737",
  "gene": "UniProtKB:P24941"
}